{
  "gene_name": "Heat shock protein HSP 90-beta",
  "term_label": "unfolded protein binding",
  "gene": "UniProtKB:P08238",
  "gene_symbol": "HSP90AB1",
  "term_id": "GO:0051082"
}